regulation of estradiol secretion [GO:2000864] (biological process) Also known as: regulation of oestradiol secretion Definition: Any process that modulates the frequency, rate or extent of estradiol secretion. Sources: GOC:sl Subtypes: GO:2000865, positive regulation of estradiol secretion [GO:2000866] Relationships: is a type of regulation of steroid hormone secretion [GO:2000831]; regulates estradiol secretion [GO:0035938]